UGG codon-amino acid adaptor activity [GO:0033416] (molecular function) Definition: A triplet codon-amino acid adaptor activity that recognizes a UGG codon. Relationships: is a type of GO:0030533 Sources: GOC:mah Note: Note that in the standard genetic code, TGG codes for tryptophan. Also known as: TGG codon-amino acid adaptor activity, tryptophan tRNA